{
  "gene_name": "Methyltransferase-like 26",
  "term_id": "UNKNOWN:0003",
  "gene_symbol": "METTL26",
  "term_label": "Unknown cellular component",
  "gene": "UniProtKB:Q96S19"
}